{
  "term_id": "GO:0005634",
  "gene_symbol": "ZNF385B",
  "gene": "UniProtKB:Q569K4",
  "term_label": "nucleus",
  "gene_name": "Zinc finger protein 385B"
}